{
  "term_label": "U6 snRNA binding",
  "gene_name": "U4_U6 small nuclear ribonucleoprotein Prp4",
  "gene": "UniProtKB:O43172",
  "gene_symbol": "PRPF4",
  "term_id": "GO:0017070"
}